{
  "term_id": "GO:0097753",
  "gene_name": "Islet cell autoantigen 1-like protein",
  "gene_symbol": "ICA1L",
  "term_label": "membrane bending",
  "gene": "UniProtKB:Q8NDH6"
}